{
  "gene": "UniProtKB:A0A2R8YD15",
  "term_label": "Unknown cellular component",
  "gene_name": "Uncharacterized protein",
  "gene_symbol": "A0A2R8YD15",
  "term_id": "UNKNOWN:0003"
}